positive regulation of aecium development [GO:0075269] (biological process) Relationships: is a type of positive regulation of spore-bearing organ development [GO:0075261]; is a type of regulation of aecium development [GO:0075268]; positively regulates aecium development [GO:0075267] Sources: GOC:pamgo_curators Definition: Any process that activates, maintains or increases the frequency, rate or extent of aecium development, a process in which a cuplike structure containing chains of aeciospores is formed.